{
  "term_label": "Unknown biological process",
  "gene": "UniProtKB:P46779",
  "gene_symbol": "RPL28",
  "gene_name": "Large ribosomal subunit protein eL28",
  "term_id": "UNKNOWN:0002"
}